{
  "gene_symbol": "GTF3C5",
  "gene": "UniProtKB:Q9Y5Q8",
  "term_label": "RNA polymerase III general transcription initiation factor activity",
  "gene_name": "General transcription factor 3C polypeptide 5",
  "term_id": "GO:0000995"
}